ribonucleoside metabolic process [GO:0009119] (biological process) Relationships: is a type of GO:0009116 Subtypes: ribonucleoside catabolic process [GO:0042454], ribonucleoside biosynthetic process [GO:0042455], purine ribonucleoside metabolic process [GO:0046128], pyrimidine ribonucleoside metabolic process [GO:0046131] Also known as: ribonucleoside metabolism Definition: The chemical reactions and pathways involving any ribonucleoside, a nucleoside in which purine or pyrimidine base is linked to a ribose (beta-D-ribofuranose) molecule. Sources: GOC:jl